{
  "term_id": "GO:0006364",
  "term_label": "rRNA processing",
  "gene_symbol": "ESF1",
  "gene": "UniProtKB:Q9H501",
  "gene_name": "ESF1 homolog"
}